{
  "gene_symbol": "OR13J1",
  "term_label": "olfactory receptor activity",
  "gene_name": "Olfactory receptor 13J1",
  "term_id": "GO:0004984",
  "gene": "UniProtKB:Q8NGT2"
}